negative regulation of T cell anergy [GO:0002668] (biological process) Definition: Any process that stops, prevents, or reduces the frequency, rate, or extent of T cell anergy. Sources: GOC:add Also known as: down regulation of T cell anergy, down-regulation of T cell anergy, downregulation of T cell anergy, negative regulation of T lymphocyte anergy, negative regulation of T-cell anergy, negative regulation of T-lymphocyte anergy, inhibition of T cell anergy Relationships: is a type of negative regulation of T cell tolerance induction [GO:0002665]; is a type of regulation of T cell anergy [GO:0002667]; is a type of negative regulation of lymphocyte anergy [GO:0002912]; negatively regulates T cell anergy [GO:0002870]